{
  "term_label": "nucleoplasm",
  "gene_symbol": "ZNF134",
  "gene": "UniProtKB:P52741",
  "gene_name": "Zinc finger protein 134",
  "term_id": "GO:0005654"
}